{
  "term_id": "GO:0000209",
  "term_label": "protein polyubiquitination",
  "gene": "UniProtKB:Q96EQ8",
  "gene_symbol": "RNF125",
  "gene_name": "E3 ubiquitin-protein ligase RNF125"
}